cell dedifferentiation [GO:0043697] (BP) Sources: GOC:dph, GOC:pg Note: Note that this term should be used to annotate gene products involved in dedifferentiation that occurs as part of a normal process, such as regeneration. It should not be used for dedifferentiation that occurs in an abnormal or disease state such as cancer. Definition: The process in which a specialized cell loses the structural or functional features that characterize it in the mature organism, or some other relatively stable phase of the organism's life history. Under certain conditions, these cells can revert back to the features of the stem cells that were their ancestors. Relationships: is a type of GO:0043696; is a type of cellular developmental process [GO:0048869] Subtypes: cell dedifferentiation involved in phenotypic switching [GO:0090678], kidney cortex tubule cell dedifferentiation [GO:0160029], hepatocyte dedifferentiation [GO:1990828]